phosphatidylinositol 3-kinase complex, class III, type I [GO:0034271] (cellular component) Relationships: is a type of phosphatidylinositol 3-kinase complex, class III [GO:0035032] Also known as: autophagy-specific phosphatidylinositol 3-kinase (PtdIns3K) complex, PtdIns-3-kinase complex I, phosphatidylinositol 3-kinase complex I Definition: A class III phosphatidylinositol 3-kinase complex that is involved in autophagy. In budding yeast, this complex consists of Vps30p, Vps34p, Apg14p and Vps15p. Note: Note that this term should not be confused with '1-phosphatidylinositol-4-phosphate 3-kinase, class IA complex; GO:0005943' or '1-phosphatidylinositol-4-phosphate 3-kinase, class IB complex ; GO:0005944'. References: PMID:11157979, PMID:16421251 Sources: GOC:ha, GOC:rb